{
  "term_label": "RNA polymerase II cis-regulatory region sequence-specific DNA binding",
  "term_id": "GO:0000978",
  "gene_name": "Transcription factor SOX-12",
  "gene_symbol": "SOX12",
  "gene": "UniProtKB:O15370"
}